regulation of secondary cell wall biogenesis [GO:2000652] (biological process) Subtypes: negative regulation of secondary cell wall biogenesis [GO:1901347], positive regulation of secondary cell wall biogenesis [GO:1901348] Relationships: is a type of regulation of cellular component biogenesis [GO:0044087]; is a type of regulation of cell wall organization or biogenesis [GO:1903338]; regulates plant-type secondary cell wall biogenesis [GO:0009834] Also known as: regulation of cellulose and pectin-containing secondary cell wall biogenesis, regulation of plant-type secondary cell wall biogenesis, regulation of secondary cell wall anabolism, regulation of secondary cell wall biosynthetic process, regulation of secondary cell wall formation, regulation of secondary cell wall synthesis Definition: Any process that modulates the frequency, rate or extent of secondary cell wall biogenesis. Sources: GOC:obol